{
  "term_label": "RNA polymerase II cis-regulatory region sequence-specific DNA binding",
  "gene_name": "Zinc finger protein 564",
  "term_id": "GO:0000978",
  "gene_symbol": "ZNF564",
  "gene": "UniProtKB:Q8TBZ8"
}